prephenate(2-) biosynthetic process [GO:1901747] (BP) Also known as: prephenate anabolism, prephenate biosynthesis, prephenate formation, prephenate synthesis, prephenate(2-) anabolism, prephenate(2-) biosynthesis, prephenate(2-) formation, prephenate(2-) synthesis Relationships: is_a GO:0043650 Definition: The chemical reactions and pathways resulting in the formation of prephenate(2-). References: PMID:16752890 Sources: GOC:TermGenie, GOC:yaf, UniPathway:UPA00120